{
  "term_label": "lysosomal membrane",
  "term_id": "GO:0005765",
  "gene": "UniProtKB:Q9NUN5",
  "gene_symbol": "LMBRD1",
  "gene_name": "Lysosomal cobalamin transport escort protein LMBD1"
}